{
  "gene": "UniProtKB:Q9UJF2",
  "gene_symbol": "RASAL2",
  "term_id": "GO:0005096",
  "term_label": "GTPase activator activity",
  "gene_name": "Ras GTPase-activating protein nGAP"
}